ornithine transport [GO:0015822] (biological process) Also known as: L-ornithine transport Relationships: is a type of amino acid transport [GO:0006865]; is a type of organic cation transport [GO:0015695]; is a type of carboxylic acid transport [GO:0046942]; is a type of nitrogen compound transport [GO:0071705] Subtypes: ornithine transmembrane import into vacuole [GO:0090455], L-ornithine transmembrane transport [GO:1903352] Definition: The directed movement of ornithine, 2,5-diaminopentanoic acid, into, out of or within a cell, or between cells, by means of some agent such as a transporter or pore. Sources: GOC:ai